{
  "gene_symbol": "TUBA1C",
  "term_id": "GO:0005525",
  "term_label": "GTP binding",
  "gene": "UniProtKB:Q9BQE3",
  "gene_name": "Tubulin alpha-1C chain"
}